{
  "term_id": "UNKNOWN:0002",
  "term_label": "Unknown biological process",
  "gene_symbol": "ZHX1-C8orf76",
  "gene": "UniProtKB:Q96EF9",
  "gene_name": "Zinc fingers and homeoboxes protein 1, isoform 2"
}